{
  "term_id": "GO:0019136",
  "gene": "UniProtKB:O00142",
  "term_label": "deoxynucleoside kinase activity",
  "gene_symbol": "TK2",
  "gene_name": "Thymidine kinase 2, mitochondrial"
}